{
  "gene_name": "Putative uncharacterized protein ENSP00000383407",
  "term_label": "Unknown biological process",
  "term_id": "UNKNOWN:0002",
  "gene_symbol": "A8MT66",
  "gene": "UniProtKB:A8MT66"
}